{
  "gene_name": "Probable tRNA (uracil-O(2)-)-methyltransferase",
  "term_id": "UNKNOWN:0003",
  "term_label": "Unknown cellular component",
  "gene_symbol": "TRMT44",
  "gene": "UniProtKB:Q8IYL2"
}